{
  "gene_name": "Histatin-1",
  "term_label": "Unknown molecular function",
  "gene_symbol": "HTN1",
  "term_id": "UNKNOWN:0001",
  "gene": "UniProtKB:P15515"
}